amino acid:potassium symporter activity [GO:0017032] (molecular function) Also known as: potassium:amino acid symporter activity Definition: Enables the transfer of a solute or solutes from one side of a membrane to the other according to the reaction: amino acid(out) + K+(out) = amino acid(in) + K+(in). Sources: GOC:ai Relationships: is a type of amino acid:monoatomic cation symporter activity [GO:0005416]; is a type of potassium ion transmembrane transporter activity [GO:0015079]